nicotinamide mononucleotide transmembrane transporter activity [GO:0015663] (molecular function) Sources: ISBN:0721662544 Definition: Enables the directed movement of nicotinamide mononucleotide into, out of or within a cell, or between cells. Nicotinamide mononucleotide is a ribonucleotide in which the nitrogenous base, nicotinamide, is in beta-n-glycosidic linkage with the c-1 position of d-ribose. It is a constituent of NAD and NADP. Relationships: is a type of nucleotide transmembrane transporter activity [GO:0015215]; is a type of GO:1901505; is part of nicotinamide mononucleotide transmembrane transport [GO:0035353] Also known as: nicotinamide ribonucleotide transmembrane transporter activity, nicotinamide mononucleotide permease activity